mesodermal cell fate specification [GO:0007501] (biological process) Relationships: is a type of cell fate specification [GO:0001708]; is part of mesodermal cell fate commitment [GO:0001710] Also known as: mesoderm cell fate specification Subtypes: axial mesodermal cell fate specification [GO:0048327], GO:0048348, lateral mesodermal cell fate specification [GO:0048377], GO:0048398 Sources: GOC:go_curators Regulation: regulated by regulation of mesodermal cell fate specification [GO:0042661]; negatively regulated by negative regulation of mesodermal cell fate specification [GO:0042662]; positively regulated by positive regulation of mesodermal cell fate specification [GO:0048337] Note: Note that this term was 'fate specification in mesoderm'. String of term was changed to correspond to format of sibling terms 'endoderm cell fate specification' and 'ectoderm cell fate specification'. Definition: The cell fate determination process in which a cell becomes capable of differentiating autonomously into a mesoderm cell in an environment that is neutral with respect to the developmental pathway; upon specification, the cell fate can be reversed.